{
  "term_id": "GO:0005249",
  "gene_name": "Potassium voltage-gated channel subfamily KQT member 3",
  "gene": "UniProtKB:O43525",
  "term_label": "voltage-gated potassium channel activity",
  "gene_symbol": "KCNQ3"
}